regulation of RNA splicing [GO:0043484] (BP) Relationships: is a type of GO:0010468; is a type of regulation of primary metabolic process [GO:0080090]; regulates GO:0008380 Definition: Any process that modulates the frequency, rate or extent of RNA splicing, the process of removing sections of the primary RNA transcript to remove sequences not present in the mature form of the RNA and joining the remaining sections to form the mature form of the RNA. Subtypes: negative regulation of RNA splicing [GO:0033119], GO:0033120, regulation of mRNA splicing, via spliceosome [GO:0048024] Sources: GOC:jl